{
  "gene": "UniProtKB:Q8N158",
  "term_id": "UNKNOWN:0001",
  "gene_name": "Glypican-2",
  "term_label": "Unknown molecular function",
  "gene_symbol": "GPC2"
}